{
  "gene_name": "Carbohydrate sulfotransferase 1",
  "term_id": "GO:0006044",
  "gene": "UniProtKB:O43916",
  "gene_symbol": "CHST1",
  "term_label": "N-acetylglucosamine metabolic process"
}